{
  "term_label": "ubiquitin-like ligase-substrate adaptor activity",
  "term_id": "GO:1990756",
  "gene_symbol": "PRAMEF25",
  "gene": "UniProtKB:A6NGN4",
  "gene_name": "PRAME family member 25"
}